{
  "gene": "UniProtKB:Q9UL41",
  "gene_name": "Paraneoplastic antigen Ma3",
  "term_label": "Unknown molecular function",
  "term_id": "UNKNOWN:0001",
  "gene_symbol": "PNMA3"
}